establishment of protein localization to chromatin [GO:0071169] (BP) Definition: The directed movement of a protein to a part of a chromosome that is organized into chromatin. Sources: GOC:mah Also known as: establishment of protein localisation to chromatin Subtypes: establishment of protein localization to euchromatin [GO:1905633] Relationships: is a type of establishment of protein localization to chromosome [GO:0070199]